{
  "gene": "UniProtKB:O14966",
  "term_id": "GO:0005802",
  "term_label": "trans-Golgi network",
  "gene_name": "Ras-related protein Rab-7L1",
  "gene_symbol": "RAB29"
}